{
  "term_id": "UNKNOWN:0002",
  "term_label": "Unknown biological process",
  "gene_symbol": "TMEM229A",
  "gene_name": "Transmembrane protein 229A",
  "gene": "UniProtKB:B2RXF0"
}